{
  "term_label": "axon guidance",
  "gene_name": "Nexilin",
  "term_id": "GO:0007411",
  "gene": "UniProtKB:Q0ZGT2",
  "gene_symbol": "NEXN"
}